{
  "gene_name": "Aquaporin-9",
  "gene": "UniProtKB:O43315",
  "term_label": "water channel activity",
  "term_id": "GO:0015250",
  "gene_symbol": "AQP9"
}